{
  "gene_name": "Leucine-rich repeat and calponin homology domain-containing protein 1",
  "gene": "UniProtKB:Q9Y2L9",
  "gene_symbol": "LRCH1",
  "term_label": "negative regulation of T cell migration",
  "term_id": "GO:2000405"
}